mitochondrial [2Fe-2S] assembly complex [GO:0099128] (cellular component) Definition: A protein complex capable of forming 2Fe-2S clusters in mitochondria. In humans it consists of ISCU, NFS1, LYRM4, NDUFAB1 and FXN. References: PMID:31101807, PMID:34660592 Relationships: is a type of mitochondrial protein-containing complex [GO:0098798]; is a type of L-cysteine desulfurase complex [GO:1990221]; is a type of iron-sulfur cluster assembly complex [GO:1990229] Also known as: mitochondrial ISCU complex, mitochondrial iron-sulfur cluster assembly complex